organelle-enclosing lipid monolayer [GO:0034646] (CC) Subtypes: chlorosome envelope [GO:0033105], GO:0034430 Sources: GOC:mah Definition: A lipid monolayer that surrounds and encloses an organelle. Relationships: is a type of GO:0110165; is part of intracellular organelle [GO:0043229]